{
  "term_id": "GO:0043171",
  "gene": "UniProtKB:Q9UKU6",
  "gene_symbol": "TRHDE",
  "term_label": "peptide catabolic process",
  "gene_name": "Thyrotropin-releasing hormone-degrading ectoenzyme"
}